{
  "gene_name": "Endothelin-1 receptor",
  "gene": "UniProtKB:P25101",
  "term_label": "plasma membrane",
  "term_id": "GO:0005886",
  "gene_symbol": "EDNRA"
}